periplasmic flagellum [GO:0055040] (cellular component) References: PMID:15175283, PMID:1624463 Sources: GOC:jid, GOC:rph Relationships: is a type of bacterial-type flagellum [GO:0009288]; is part of GO:0042597 Definition: Flagellar filaments located in the periplasmic space; characterized in spirochetes, in which they are essential for shape and motility. Composed of a core surrounded by two sheath layers, the flagella rotate to allow migration of the cell through viscous media, which would not be possible using external flagella.